{
  "gene": "UniProtKB:P49841",
  "gene_symbol": "GSK3B",
  "term_label": "positive regulation of proteasomal ubiquitin-dependent protein catabolic process",
  "term_id": "GO:0032436",
  "gene_name": "Glycogen synthase kinase-3 beta"
}